{
  "gene": "UniProtKB:Q6PCT2",
  "term_label": "Unknown cellular component",
  "term_id": "UNKNOWN:0003",
  "gene_symbol": "FBXL19",
  "gene_name": "F-box_LRR-repeat protein 19"
}